{
  "gene_name": "Mitochondrial 2-oxodicarboxylate carrier",
  "gene_symbol": "SLC25A21",
  "term_label": "Unknown cellular component",
  "term_id": "UNKNOWN:0003",
  "gene": "UniProtKB:Q9BQT8"
}